positive regulation of axon extension [GO:0045773] (biological process) Subtypes: GO:0048691, GO:0048842 Definition: Any process that activates or increases the frequency, rate or extent of axon extension. Sources: GOC:go_curators Also known as: up regulation of axon extension, up-regulation of axon extension, upregulation of axon extension, activation of axon extension, stimulation of axon extension Relationships: is a type of positive regulation of cell growth [GO:0030307]; is a type of regulation of axon extension [GO:0030516]; is a type of positive regulation of developmental growth [GO:0048639]; is a type of positive regulation of axonogenesis [GO:0050772]; positively regulates GO:0048675